{
  "gene_symbol": "COMMD2",
  "term_id": "UNKNOWN:0003",
  "gene_name": "COMM domain-containing protein 2",
  "gene": "UniProtKB:Q86X83",
  "term_label": "Unknown cellular component"
}